{
  "gene_symbol": "CTAG1A",
  "term_label": "Unknown cellular component",
  "term_id": "UNKNOWN:0003",
  "gene": "UniProtKB:P78358",
  "gene_name": "Cancer_testis antigen 1"
}